{
  "term_label": "Unknown biological process",
  "gene": "UniProtKB:Q2TAM9",
  "gene_name": "Tumor suppressor candidate gene 1 protein",
  "gene_symbol": "TUSC1",
  "term_id": "UNKNOWN:0002"
}